{
  "gene_symbol": "LRRC63",
  "term_id": "GO:0035556",
  "term_label": "intracellular signal transduction",
  "gene": "UniProtKB:Q05C16",
  "gene_name": "Leucine-rich repeat-containing protein 63"
}